{
  "gene_name": "Arf-GAP with coiled-coil, ANK repeat and PH domain-containing protein 1",
  "term_label": "Unknown molecular function",
  "term_id": "UNKNOWN:0001",
  "gene_symbol": "ACAP1",
  "gene": "UniProtKB:Q15027"
}